DNA-templated transcription initiation [GO:0006352] (biological process) References: PMID:18280161 Sources: GOC:jid, GOC:txnOH Definition: The initial step of transcription, consisting of the assembly of the RNA polymerase preinitiation complex (PIC) at a gene promoter, as well as the formation of the first few bonds of the RNA transcript. Transcription initiation includes abortive initiation events, which occur when the first few nucleotides are repeatedly synthesized and then released, and ends when promoter clearance takes place. Subtypes: GO:0006361, GO:0006367, transcription initiation at RNA polymerase III promoter [GO:0006384], GO:0006391 Regulation: RO_0002211 by GO:2000142; negatively regulated by negative regulation of DNA-templated transcription initiation [GO:2000143]; RO_0002213 by positive regulation of DNA-templated transcription initiation [GO:2000144] Note: Note that promoter clearance is represented as a separate step, not part_of either initiation or elongation. Also known as: DNA-dependent RNA polymerase complex assembly at promoter, DNA-dependent transcription, initiation, DNA-templated transcription, initiation, initiation of DNA-dependent transcription, initiation of transcription, DNA-dependent, transcription initiation from bacterial-type RNA polymerase promoter, transcription initiation factor activity, transcription initiation, DNA-dependent Relationships: is a type of RNA biosynthetic process [GO:0032774]; is part of DNA-templated transcription [GO:0006351]